posterior semicircular canal development [GO:0060874] (biological process) Definition: The progession of the posterior semicircular canal from its initial formation to the mature structure. Sources: GOC:dph, GOC:sdb_2009, GOC:tb Relationships: is a type of semicircular canal development [GO:0060872]